negative regulation of fibroblast growth factor production [GO:0090272] (biological process) Relationships: is a type of negative regulation of cytokine production [GO:0001818]; is a type of regulation of fibroblast growth factor production [GO:0090270]; negatively regulates GO:0090269 Definition: Any process that decreases the rate, frequency or extent of the appearance of a fibroblast growth factor due to biosynthesis or secretion following a cellular stimulus, resulting in an increase in its intracellular or extracellular levels. Sources: GOC:BHF